negative regulation of natural killer cell mediated immunity [GO:0002716] (BP) Relationships: is a type of negative regulation of lymphocyte mediated immunity [GO:0002707]; is a type of regulation of natural killer cell mediated immunity [GO:0002715]; is a type of GO:0045824; negatively regulates natural killer cell mediated immunity [GO:0002228] Subtypes: negative regulation of natural killer cell cytokine production [GO:0002728], GO:0002856, GO:0045953 Also known as: down regulation of natural killer cell mediated immunity, down-regulation of natural killer cell mediated immunity, downregulation of natural killer cell mediated immunity, negative regulation of NK cell mediated immunity, inhibition of natural killer cell mediated immunity, negative regulation of NK cell activity, negative regulation of natural killer cell activity Definition: Any process that stops, prevents, or reduces the frequency, rate, or extent of natural killer cell mediated immunity. Sources: GOC:add